{
  "term_label": "cell migration",
  "gene_symbol": "KDR",
  "gene": "UniProtKB:P35968",
  "term_id": "GO:0016477",
  "gene_name": "Vascular endothelial growth factor receptor 2"
}